{
  "term_label": "endoplasmic reticulum",
  "term_id": "GO:0005783",
  "gene_symbol": "EDEM3",
  "gene_name": "ER degradation-enhancing alpha-mannosidase-like protein 3",
  "gene": "UniProtKB:Q9BZQ6"
}